{
  "term_id": "GO:0035725",
  "gene": "UniProtKB:P78348",
  "gene_name": "Acid-sensing ion channel 1",
  "gene_symbol": "ASIC1",
  "term_label": "sodium ion transmembrane transport"
}